{
  "term_id": "GO:0005737",
  "term_label": "cytoplasm",
  "gene_symbol": "AGO3",
  "gene": "UniProtKB:Q9H9G7",
  "gene_name": "Protein argonaute-3"
}